substrate-dependent cell migration, cell contraction [GO:0006932] (biological process) Definition: The translocation of the cell body forward during cell migration, mediated by tractional force on its substrate and tension in the cortical cytoskeleton. Adhesions transmit propulsive forces and serve as traction points over which the cell moves. Also known as: substrate-bound cell migration, cell contraction Relationships: is a type of cytoplasmic actin-based contraction involved in cell motility [GO:0060327]; is part of ameboidal-type cell migration [GO:0001667]; is part of GO:0006929 References: PMID:11944043, PMID:14657486 Sources: ISBN:0815316194